{
  "term_label": "positive regulation of actin filament polymerization",
  "gene": "UniProtKB:Q6UXY1",
  "gene_name": "Brain-specific angiogenesis inhibitor 1-associated protein 2-like protein 2",
  "term_id": "GO:0030838",
  "gene_symbol": "BAIAP2L2"
}